{
  "gene": "UniProtKB:P17081",
  "term_label": "plasma membrane",
  "gene_name": "Rho-related GTP-binding protein RhoQ",
  "term_id": "GO:0005886",
  "gene_symbol": "RHOQ"
}